{
  "gene_name": "Dermatan-sulfate epimerase",
  "term_id": "GO:0050655",
  "term_label": "dermatan sulfate proteoglycan metabolic process",
  "gene_symbol": "DSE",
  "gene": "UniProtKB:Q9UL01"
}